mesonephric glomerular epithelial cell differentiation [GO:0061250] (biological process) Sources: GOC:mtg_kidney_jan10 Definition: The process in which a relatively unspecialized cell acquires specialized features of a mesonephric glomerular epithelial cell. Mesonephric glomerular epithelial cells are specialized epithelial cells that form part of the mesonephric glomerulus; there are two types, mesonephric glomerular parietal epithelial cells and mesonephric glomerular visceral epithelial cells. Relationships: is a type of cell differentiation involved in mesonephros development [GO:0061208]; is a type of glomerular epithelial cell differentiation [GO:0072311]; is part of mesonephric glomerular epithelium development [GO:0061232] Subtypes: mesonephric glomerular parietal epithelial cell differentiation [GO:0061253], mesonephric podocyte differentiation [GO:0061256]